{
  "gene": "UniProtKB:O75888",
  "gene_symbol": "TNFSF13",
  "term_id": "GO:0005615",
  "term_label": "extracellular space",
  "gene_name": "Tumor necrosis factor ligand superfamily member 13"
}